{
  "gene": "UniProtKB:P22607",
  "gene_name": "Fibroblast growth factor receptor 3",
  "term_id": "GO:0008543",
  "gene_symbol": "FGFR3",
  "term_label": "fibroblast growth factor receptor signaling pathway"
}